{
  "term_label": "vacuolar transport",
  "term_id": "GO:0007034",
  "gene_name": "Protein CLEC16A",
  "gene": "UniProtKB:Q2KHT3",
  "gene_symbol": "CLEC16A"
}